{
  "term_label": "regulation of transcription by RNA polymerase II",
  "gene": "UniProtKB:Q76KX8",
  "gene_symbol": "ZNF534",
  "term_id": "GO:0006357",
  "gene_name": "Zinc finger protein 534"
}